{
  "term_id": "GO:0004420",
  "gene_name": "3-hydroxy-3-methylglutaryl-coenzyme A reductase",
  "term_label": "hydroxymethylglutaryl-CoA reductase (NADPH) activity",
  "gene": "UniProtKB:P04035",
  "gene_symbol": "HMGCR"
}